{
  "gene_symbol": "RPE",
  "term_id": "GO:0005829",
  "gene_name": "Ribulose-phosphate 3-epimerase",
  "term_label": "cytosol",
  "gene": "UniProtKB:Q96AT9"
}